{
  "term_label": "nucleus",
  "gene_symbol": "ZNF563",
  "gene_name": "Zinc finger protein 563",
  "term_id": "GO:0005634",
  "gene": "UniProtKB:Q8TA94"
}